{
  "gene_symbol": "ZNF607",
  "gene_name": "Zinc finger protein 607",
  "term_label": "DNA-binding transcription factor activity, RNA polymerase II-specific",
  "term_id": "GO:0000981",
  "gene": "UniProtKB:Q96SK3"
}